{
  "term_id": "GO:0006508",
  "gene_symbol": "LNPEP",
  "gene": "UniProtKB:Q9UIQ6",
  "term_label": "proteolysis",
  "gene_name": "Leucyl-cystinyl aminopeptidase"
}